{
  "gene": "UniProtKB:P01567",
  "term_id": "GO:0006959",
  "gene_name": "Interferon alpha-7",
  "gene_symbol": "IFNA7",
  "term_label": "humoral immune response"
}